{
  "term_label": "cellular response to lipopolysaccharide",
  "gene_symbol": "IL36G",
  "term_id": "GO:0071222",
  "gene": "UniProtKB:Q9NZH8",
  "gene_name": "Interleukin-36 gamma"
}